regulation of miRNA metabolic process [GO:2000628] (biological process) Also known as: regulation of microRNA metabolic process Sources: GOC:dph Relationships: is a type of regulation of RNA metabolic process [GO:0051252]; regulates miRNA metabolic process [GO:0010586] Subtypes: regulation of miRNA transcription [GO:1902893], GO:2000625, negative regulation of miRNA metabolic process [GO:2000629], GO:2000630 Definition: Any process that modulates the frequency, rate or extent of miRNA metabolic process.